{
  "gene": "UniProtKB:Q8NH76",
  "term_id": "UNKNOWN:0002",
  "term_label": "Unknown biological process",
  "gene_name": "Olfactory receptor 56B4",
  "gene_symbol": "OR56B4"
}